{
  "term_id": "GO:0009986",
  "gene_name": "Epidermal growth factor-like protein 8",
  "term_label": "cell surface",
  "gene": "UniProtKB:Q99944",
  "gene_symbol": "EGFL8"
}